{
  "gene_name": "Protein FAM25A",
  "gene": "UniProtKB:B3EWG3",
  "term_label": "Unknown molecular function",
  "gene_symbol": "FAM25A",
  "term_id": "UNKNOWN:0001"
}